{
  "term_id": "GO:0005739",
  "gene_name": "Protein Mpv17",
  "gene": "UniProtKB:P39210",
  "gene_symbol": "MPV17",
  "term_label": "mitochondrion"
}